{
  "term_label": "Unknown biological process",
  "gene_name": "Uncharacterized protein CFAP92",
  "gene": "UniProtKB:Q9ULG3",
  "gene_symbol": "CFAP92",
  "term_id": "UNKNOWN:0002"
}